negative regulation of quinolinate biosynthetic process [GO:1904985] (biological process) Definition: Any process that stops, prevents or reduces the frequency, rate or extent of quinolinate biosynthetic process. References: PMID:12140278, PMID:19843166 Sources: GOC:PARL, GOC:TermGenie, GOC:bf, GO_REF:0000058 Also known as: down regulation of quinolinate anabolism, down regulation of quinolinate biosynthesis, down regulation of quinolinate biosynthetic process, down regulation of quinolinate formation, down regulation of quinolinate synthesis, down-regulation of quinolinate anabolism, down-regulation of quinolinate biosynthesis, down-regulation of quinolinate biosynthetic process, down-regulation of quinolinate formation, down-regulation of quinolinate synthesis, downregulation of quinolinate anabolism, downregulation of quinolinate biosynthesis, downregulation of quinolinate biosynthetic process, downregulation of quinolinate formation, downregulation of quinolinate synthesis, negative regulation of quinolinate anabolism, negative regulation of quinolinate biosynthesis, negative regulation of quinolinate formation, negative regulation of quinolinate synthesis, inhibition of quinolinate anabolism, inhibition of quinolinate biosynthesis, inhibition of quinolinate biosynthetic process, inhibition of quinolinate formation, inhibition of quinolinate synthesis Relationships: is a type of negative regulation of biosynthetic process [GO:0009890]; is a type of negative regulation of small molecule metabolic process [GO:0062014]; is a type of regulation of quinolinate biosynthetic process [GO:1904984]; negatively regulates GO:0019805